{
  "gene_symbol": "HDAC7",
  "term_label": "histone deacetylase complex",
  "gene": "UniProtKB:Q8WUI4",
  "gene_name": "Histone deacetylase 7",
  "term_id": "GO:0000118"
}